desmosome organization [GO:0002934] (biological process) Definition: A process that is carried out at the cellular level which results in the assembly, arrangement of constituent parts, or disassembly of a desmosome. A desmosome is a patch-like intercellular junction found in vertebrate tissues, consisting of parallel zones of two cell membranes, separated by an space of 25-35 nm, and having dense fibrillar plaques in the subjacent cytoplasm. Subtypes: desmosome assembly [GO:0002159], desmosome maintenance [GO:0002160], GO:0035921 Sources: GOC:hjd Relationships: is a type of GO:0045216